regulation of phosphorelay signal transduction system [GO:0070297] (biological process) Definition: Any process that modulates the frequency, rate or extent of signal transduction via a phosphorelay signal transduction system. Also known as: regulation of histidyl-aspartyl phosphorelay, regulation of two-component signal transduction system, regulation of two-component signal transduction system (phosphorelay) Subtypes: regulation of ethylene-activated signaling pathway [GO:0010104], negative regulation of phosphorelay signal transduction system [GO:0070298], positive regulation of phosphorelay signal transduction system [GO:0070299] Relationships: is a type of regulation of intracellular signal transduction [GO:1902531]; regulates phosphorelay signal transduction system [GO:0000160] Sources: GOC:mah